{
  "gene": "UniProtKB:Q96EE3",
  "gene_symbol": "SEH1L",
  "term_label": "nuclear pore outer ring",
  "gene_name": "Nucleoporin SEH1",
  "term_id": "GO:0031080"
}